{
  "gene_symbol": "IL13RA2",
  "gene": "UniProtKB:Q14627",
  "term_id": "GO:0019955",
  "gene_name": "Interleukin-13 receptor subunit alpha-2",
  "term_label": "cytokine binding"
}